{
  "gene_symbol": "NR1H3",
  "term_label": "negative regulation of transcription by RNA polymerase II",
  "gene_name": "Oxysterols receptor LXR-alpha",
  "term_id": "GO:0000122",
  "gene": "UniProtKB:Q13133"
}